{
  "term_label": "proteolysis",
  "gene": "UniProtKB:Q96KN2",
  "gene_symbol": "CNDP1",
  "gene_name": "Beta-Ala-His dipeptidase",
  "term_id": "GO:0006508"
}